{
  "gene_name": "DEP domain-containing protein 1A",
  "term_label": "transcription repressor complex",
  "gene": "UniProtKB:Q5TB30",
  "gene_symbol": "DEPDC1",
  "term_id": "GO:0017053"
}